{
  "term_label": "actin cytoskeleton organization",
  "gene": "UniProtKB:Q13643",
  "gene_name": "Four and a half LIM domains protein 3",
  "term_id": "GO:0030036",
  "gene_symbol": "FHL3"
}